{
  "term_id": "GO:0061630",
  "gene": "UniProtKB:Q75N03",
  "gene_name": "E3 ubiquitin-protein ligase Hakai",
  "term_label": "ubiquitin protein ligase activity",
  "gene_symbol": "CBLL1"
}